{
  "gene_name": "Pantothenate kinase 1",
  "gene": "UniProtKB:Q8TE04",
  "gene_symbol": "PANK1",
  "term_id": "GO:0005829",
  "term_label": "cytosol"
}